{
  "gene_name": "Adenosine deaminase domain-containing protein 1",
  "gene_symbol": "ADAD1",
  "gene": "UniProtKB:Q96M93",
  "term_id": "GO:0003726",
  "term_label": "double-stranded RNA adenosine deaminase activity"
}